{
  "term_id": "GO:0060048",
  "gene_symbol": "MYL3",
  "gene_name": "Myosin light chain 3",
  "term_label": "cardiac muscle contraction",
  "gene": "UniProtKB:P08590"
}